{
  "gene_name": "Putative zinc finger protein 705EP",
  "term_label": "regulation of transcription by RNA polymerase II",
  "gene": "UniProtKB:A8MWA4",
  "term_id": "GO:0006357",
  "gene_symbol": "ZNF705EP"
}